{
  "gene": "UniProtKB:Q86W28",
  "term_label": "Unknown molecular function",
  "gene_name": "NACHT, LRR and PYD domains-containing protein 8",
  "term_id": "UNKNOWN:0001",
  "gene_symbol": "NLRP8"
}